{
  "term_label": "Dbf4-dependent protein kinase complex",
  "term_id": "GO:0031431",
  "gene_name": "Protein DBF4 homolog A",
  "gene_symbol": "DBF4",
  "gene": "UniProtKB:Q9UBU7"
}